{
  "gene": "UniProtKB:Q8TCJ0",
  "gene_name": "F-box only protein 25",
  "term_id": "UNKNOWN:0001",
  "gene_symbol": "FBXO25",
  "term_label": "Unknown molecular function"
}